{
  "gene_symbol": "SSR3",
  "term_label": "endoplasmic reticulum",
  "gene_name": "Translocon-associated protein subunit gamma",
  "term_id": "GO:0005783",
  "gene": "UniProtKB:Q9UNL2"
}